postsynaptic Golgi apparatus [GO:0150051] (cellular component) Also known as: Golgi outpost References: PMID:23838184 Sources: GOC:aruk, GOC:bc Definition: The network of the Golgi apparatus structures located within the postsynapse. Relationships: is a type of GO:0005794; is part of GO:0098794